{
  "gene_symbol": "CAV3",
  "gene": "UniProtKB:P56539",
  "term_label": "regulation of cytosolic calcium ion concentration",
  "term_id": "GO:0051480",
  "gene_name": "Caveolin-3"
}